slime layer [GO:0030114] (cellular component) Definition: A slime layer is an easily removed, diffuse, unorganized layer of extracellular material that surrounds a cell. Specifically this consists mostly of exopolysaccharides, glycoproteins, and glycolipids. Relationships: is a type of glycocalyx [GO:0030112] Sources: GOC:mlg, Wikipedia:Slime_layer